response to pheromone triggering conjugation with cellular fusion [GO:0000749] (biological process) Definition: Any process that results in a change in state or activity of a cell or an organism (in terms of movement, secretion, enzyme production, gene expression, etc.) as a result of a pheromone stimulus that positively regulates the process of conjugation with cellular fusion. An example of this process is found in Saccharomyces cerevisiae. Sources: GOC:clt Relationships: is a type of cellular response to pheromone [GO:0071444]; positively regulates conjugation with cellular fusion [GO:0000747] Also known as: response to pheromone during conjugation with cellular fusion